{
  "gene": "UniProtKB:O60921",
  "term_id": "GO:0035861",
  "term_label": "site of double-strand break",
  "gene_name": "Checkpoint protein HUS1",
  "gene_symbol": "HUS1"
}